symbiont-mediated disruption of host chloroplast thylakoid [GO:0033658] (biological process) Sources: GOC:pamgo_curators Relationships: is a type of symbiont-mediated disruption of host cellular anatomical structure [GO:0052008] Definition: The process in which an organism effects a change that impairs the structure or function of the host cell chloroplast thylakoid. The host is defined as the larger of the organisms involved in a symbiotic interaction. Also known as: disruption by symbiont of host chloroplast thylakoid, modification by symbiont of host chloroplast thylakoid